{
  "term_label": "G-protein beta/gamma-subunit complex binding",
  "gene_name": "Guanine nucleotide-binding protein subunit alpha-11",
  "gene_symbol": "GNA11",
  "gene": "UniProtKB:P29992",
  "term_id": "GO:0031683"
}